{
  "gene": "UniProtKB:P47710",
  "gene_name": "Alpha-S1-casein",
  "gene_symbol": "CSN1S1",
  "term_id": "GO:0005615",
  "term_label": "extracellular space"
}